{
  "gene_name": "Eukaryotic translation initiation factor 4 gamma 3",
  "term_id": "GO:0003743",
  "gene_symbol": "EIF4G3",
  "term_label": "translation initiation factor activity",
  "gene": "UniProtKB:O43432"
}